epinephrine catabolic process [GO:0042419] (biological process) Definition: The chemical reactions and pathways resulting in the breakdown of epinephrine, a hormone produced by the medulla of the adrenal glands that increases heart activity, improves the power and prolongs the action of muscles, and increases the rate and depth of breathing. It is synthesized by the methylation of norepinephrine. Sources: GOC:jl, ISBN:0192801023, ISBN:0198506732 Also known as: adrenaline catabolic process, adrenaline catabolism, epinephrine breakdown, epinephrine catabolism, epinephrine degradation Relationships: is a type of epinephrine metabolic process [GO:0042414]; is a type of catecholamine catabolic process [GO:0042424] Subtypes: GO:0001995